{
  "gene_symbol": "OR8H3",
  "term_id": "GO:0007608",
  "term_label": "sensory perception of smell",
  "gene_name": "Olfactory receptor 8H3",
  "gene": "UniProtKB:Q8N146"
}